{
  "gene": "UniProtKB:Q969Q6",
  "term_id": "GO:0045579",
  "term_label": "positive regulation of B cell differentiation",
  "gene_symbol": "PPP2R3C",
  "gene_name": "Serine_threonine-protein phosphatase 2A regulatory subunit B'' subunit gamma"
}